{
  "gene": "UniProtKB:Q5VZI3",
  "term_id": "UNKNOWN:0003",
  "gene_symbol": "TMEM268",
  "gene_name": "Transmembrane protein 268",
  "term_label": "Unknown cellular component"
}